UDP-N-acetylglucosamine metabolic process [GO:0006047] (biological process) Definition: The chemical reactions and pathways involving UDP-N-acetylglucosamine, a substance composed of N-acetylglucosamine, a common structural unit of oligosaccharides, in glycosidic linkage with uridine diphosphate. Also known as: UDP-N-acetylglucosamine metabolism Relationships: is a type of GO:0006040; is a type of nucleotide-sugar metabolic process [GO:0009225] Sources: GOC:ai Subtypes: UDP-N-acetylglucosamine biosynthetic process [GO:0006048]